{
  "gene_symbol": "GIP",
  "term_label": "response to starvation",
  "term_id": "GO:0042594",
  "gene": "UniProtKB:P09681",
  "gene_name": "Gastric inhibitory polypeptide"
}